{
  "gene_name": "UDP-glucuronosyltransferase 1A5",
  "gene": "UniProtKB:P35504",
  "term_label": "sterol metabolic process",
  "term_id": "GO:0016125",
  "gene_symbol": "UGT1A5"
}